{
  "gene_name": "Putative transmembrane protein ZNF593OS",
  "gene": "UniProtKB:A0A0U1RRA0",
  "term_id": "UNKNOWN:0002",
  "term_label": "Unknown biological process",
  "gene_symbol": "ZNF593OS"
}